{
  "gene_name": "Regulating synaptic membrane exocytosis protein 1",
  "term_id": "GO:0042734",
  "gene": "UniProtKB:Q86UR5",
  "gene_symbol": "RIMS1",
  "term_label": "presynaptic membrane"
}